galactarate transmembrane transporter activity [GO:1902301] (molecular function) Also known as: galactaric acid anion transmembrane transporter activity, D-galactarate transmembrane transporter activity Definition: Enables the transfer of galactaric acid anion (galactarate) from one side of a membrane to the other. Relationships: is a type of aldarate transmembrane transporter activity [GO:0042876]; is part of galactarate transmembrane transport [GO:1902300] Sources: GOC:TermGenie, GOC:pr